{
  "term_label": "regulation of transcription by RNA polymerase II",
  "term_id": "GO:0006357",
  "gene_name": "Homeobox protein aristaless-like 3",
  "gene_symbol": "ALX3",
  "gene": "UniProtKB:O95076"
}